{
  "gene": "UniProtKB:Q9Y2V7",
  "gene_symbol": "COG6",
  "term_label": "intra-Golgi vesicle-mediated transport",
  "term_id": "GO:0006891",
  "gene_name": "Conserved oligomeric Golgi complex subunit 6"
}